{
  "gene_symbol": "MECR",
  "term_id": "GO:0006631",
  "gene_name": "Enoyl-[acyl-carrier-protein] reductase, mitochondrial",
  "gene": "UniProtKB:Q9BV79",
  "term_label": "fatty acid metabolic process"
}